{
  "term_label": "cytoplasm",
  "gene": "UniProtKB:P0C7W6",
  "gene_name": "Coiled-coil domain-containing protein 172",
  "term_id": "GO:0005737",
  "gene_symbol": "CCDC172"
}